{
  "gene_symbol": "A0A6Q8PFC9",
  "term_label": "Unknown biological process",
  "term_id": "UNKNOWN:0002",
  "gene_name": "Uncharacterized protein",
  "gene": "UniProtKB:A0A6Q8PFC9"
}